{
  "term_label": "alpha-amylase activity",
  "gene_symbol": "AMY1B",
  "term_id": "GO:0004556",
  "gene_name": "Alpha-amylase 1B",
  "gene": "UniProtKB:P0DTE7"
}